alkylglycerone kinase activity [GO:0047650] (molecular function) Also known as: ATP:O-alkylglycerone phosphotransferase activity, alkyldihydroxyacetone kinase (phosphorylating), alkyldihydroxyacetone kinase activity Definition: Catalysis of the reaction: O-alkylglycerone + ATP = O-alkylglycerone phosphate + ADP + 2 H+. Relationships: is a type of kinase activity [GO:0016301]; is a type of phosphotransferase activity, alcohol group as acceptor [GO:0016773] Sources: EC:2.7.1.84, RHEA:23088